isoflavone 7-O-glucosyltransferase activity [GO:0050004] (molecular function) Also known as: UDP-glucose:isoflavone 7-O-beta-D-glucosyltransferase activity, UDPglucose-flavonoid 7-O-glucosyltransferase activity, UDPglucose:isoflavone 7-O-beta-D-glucosyltransferase activity, UDPglucose:isoflavone 7-O-glucosyltransferase activity, uridine diphosphoglucose-isoflavone 7-O-glucosyltransferase activity Definition: Catalysis of the reaction: UDP-glucose + isoflavone = UDP + isoflavone 7-O-beta-D-glucoside. Relationships: is a type of UDP-glucosyltransferase activity [GO:0035251] Sources: EC:2.4.1.170, MetaCyc:ISOFLAVONE-7-O-GLUCOSYLTRANSFERASE-RXN